intramolecular phosphotransferase activity [GO:0016868] (molecular function) Also known as: intramolecular transferase activity, phosphotransferases, phosphomutase activity, phosphotransferase activity, with regeneration of donors, apparently catalyzing intramolecular transfers Relationships: is a type of GO:0016866 Definition: Catalysis of the transfer of a phosphate group from one position to another within a single molecule. Subtypes: GO:0004082, phosphoacetylglucosamine mutase activity [GO:0004610], phosphoglucomutase activity [GO:0004614], GO:0004615, GO:0004619, beta-phosphoglucomutase activity [GO:0008801], phosphoglucosamine mutase activity [GO:0008966], D-sedoheptulose 7-phosphate isomerase activity [GO:0008968], phosphopentomutase activity [GO:0008973], phosphoenolpyruvate mutase activity [GO:0050188] Sources: GOC:mah